symbiont-mediated suppression of defense-related host salicylic acid-mediated signal transduction pathway [GO:0052003] (biological process) Also known as: negative regulation by organism of defense-related salicylic acid-mediated signal transduction pathway of other organism involved in symbiotic interaction, negative regulation by organism of salicylic acid-mediated defense response of other organism involved in symbiotic interaction, disruption of defense-related host salicylic acid-mediated signal transduction pathway, down regulation by symbiont of defense-related host salicylic acid-mediated signal transduction pathway, down regulation by symbiont of host salicylic acid-mediated defense response, down-regulation by symbiont of defense-related host salicylic acid-mediated signal transduction pathway, down-regulation by symbiont of host salicylic acid-mediated defense response, downregulation by symbiont of defense-related host salicylic acid-mediated signal transduction pathway, downregulation by symbiont of host salicylic acid-mediated defense response, negative modulation by organism of defense-related host SA-mediated signal transduction pathway, negative modulation by organism of defense-related host salicylic acid-mediated signal transduction pathway, negative regulation by organism of defense-related host SA-mediated signal transduction pathway, negative regulation by symbiont of defense-related host salicylic acid-mediated signal transduction pathway, negative regulation by symbiont of host salicylic acid-mediated defense response, negative regulation of host SA-mediated defense response, suppression by organism of host salicylic acid-mediated defense response, suppression by symbiont of defense-related host salicylic acid-mediated signal transduction pathway, suppression of host SA mediated defense response, inhibition by symbiont of defense-related host salicylic acid-mediated signal transduction pathway, inhibition by symbiont of host salicylic acid-mediated defense response Subtypes: effector-mediated suppression of host salicylic acid-mediated innate immune signaling [GO:0140502] Relationships: is a type of GO:0052081; negatively regulates systemic acquired resistance [GO:0009627]; negatively regulates systemic acquired resistance, salicylic acid mediated signaling pathway [GO:0009862] Sources: GOC:mtg_pamgo_17jul06 Definition: A process in which a virus interferes with, inhibits or disrupts a host salicylic acid-mediated signal transduction pathways during the host defense response. The host is defined as the larger of the organisms involved in a symbiotic interaction.